{
  "gene": "UniProtKB:Q6SPF0",
  "term_id": "GO:0000122",
  "term_label": "negative regulation of transcription by RNA polymerase II",
  "gene_symbol": "SAMD1",
  "gene_name": "Sterile alpha motif domain-containing protein 1"
}